iodotyrosine deiodinase activity [GO:0140616] (molecular function) Also known as: iodide peroxidase-tyrosine iodinase activity, iodotyrosine deiodase activity, monoiodotyrosine deiodinase activity, tyrosine iodinase activity Relationships: is_a oxidoreductase activity, acting on X-H and Y-H to form an X-Y bond [GO:0046992] Definition: Catalyzes the reaction: 2 iodide + L-tyrosine + 2 NADP+ = 3,5-diiodo-L-tyrosine + H+ + 2 NADPH. Note that this activity has only been demonstrated in the direction of 3-deiodination. 3-bromo-L-tyrosine and 3-chloro-L-tyrosine can also be used as substrates. References: PMID:15289438, PMID:18434651, PMID:25395621, PMID:27643701 Sources: RHEA:32479